{
  "gene": "UniProtKB:Q15761",
  "gene_name": "Neuropeptide Y receptor type 5",
  "term_id": "GO:0001601",
  "term_label": "peptide YY receptor activity",
  "gene_symbol": "NPY5R"
}